negative regulation of glycolytic process through fructose-6-phosphate [GO:1904539] (biological process) Definition: Any process that stops, prevents or reduces the frequency, rate or extent of glycolytic process through fructose-6-phosphate. Sources: GOC:TermGenie, GOC:dph, GO_REF:0000058, ISBN:0201090910, ISBN:0879010479 Also known as: down regulation of glycolysis through fructose-6-phosphate, down regulation of glycolytic process through fructose-6-phosphate, down-regulation of glycolysis through fructose-6-phosphate, down-regulation of glycolytic process through fructose-6-phosphate, downregulation of glycolysis through fructose-6-phosphate, downregulation of glycolytic process through fructose-6-phosphate, negative regulation of glycolysis through fructose-6-phosphate, inhibition of glycolysis through fructose-6-phosphate, inhibition of glycolytic process through fructose-6-phosphate Relationships: is a type of negative regulation of glycolytic process [GO:0045820]; is a type of GO:1904538; negatively regulates glycolytic process through fructose-6-phosphate [GO:0061615]